{
  "gene_name": "Fatty acid CoA ligase Acsl3",
  "gene": "UniProtKB:O95573",
  "term_id": "GO:0005811",
  "term_label": "lipid droplet",
  "gene_symbol": "ACSL3"
}